IgE receptor activity [GO:0019767] (molecular function) Subtypes: high-affinity IgE receptor activity [GO:0019768], GO:0019769 Definition: Combining with an immunoglobulin of the IgE isotype via the Fc region, and transmitting the signal from one side of the membrane to the other to initiate a change in cell activity. Relationships: is a type of immunoglobulin receptor activity [GO:0019763]; BFO_0000050 Fc-epsilon receptor signaling pathway [GO:0038095]; BFO_0000051 IgE binding [GO:0019863] Sources: GOC:add, GOC:signaling, ISBN:0781735149